{
  "term_label": "cell surface receptor protein tyrosine kinase signaling pathway",
  "gene_name": "Receptor-type tyrosine-protein kinase FLT3",
  "gene_symbol": "FLT3",
  "gene": "UniProtKB:P36888",
  "term_id": "GO:0007169"
}